{
  "term_id": "GO:0003823",
  "gene_name": "Immunoglobulin lambda constant 2",
  "gene_symbol": "IGLC2",
  "gene": "UniProtKB:P0DOY2",
  "term_label": "antigen binding"
}